{
  "term_id": "UNKNOWN:0001",
  "term_label": "Unknown molecular function",
  "gene_name": "Charged multivesicular body protein 5",
  "gene": "UniProtKB:Q9NZZ3",
  "gene_symbol": "CHMP5"
}